{
  "gene_name": "Olfactory receptor 6C76",
  "gene": "UniProtKB:A6NM76",
  "term_label": "Unknown biological process",
  "gene_symbol": "OR6C76",
  "term_id": "UNKNOWN:0002"
}